vitelline envelope [GO:0060388] (cellular component) Definition: A glycoprotein-based structure that lies outside the plasma membrane and surrounds the egg before fertilization. Relationships: is a type of egg coat [GO:0035805] Sources: GOC:dph, ISBN:0878932437 Also known as: fertilization membrane